negative regulation of microglial cell activation [GO:1903979] (biological process) Definition: Any process that stops, prevents or reduces the frequency, rate or extent of microglial cell activation. Relationships: is a type of negative regulation of macrophage activation [GO:0043031]; is a type of negative regulation of neuroinflammatory response [GO:0150079]; is a type of regulation of microglial cell activation [GO:1903978]; RO_0002212 microglial cell activation [GO:0001774] Also known as: down regulation of microglial cell activation, down-regulation of microglial cell activation, downregulation of microglial cell activation, inhibition of microglial cell activation References: PMID:19100238 Sources: GOC:BHF, GOC:TermGenie, GOC:nc, GO_REF:0000058